nicotinate-N-glucosyltransferase activity [GO:0050139] (molecular function) Sources: EC:2.4.1.196, RHEA:19437 Definition: Catalysis of the reaction: nicotinate + UDP-D-glucose = N-(beta-D-glucosyl)nicotinate + UDP. Relationships: is a type of UDP-glucosyltransferase activity [GO:0035251] Also known as: nicotinate glucosyltransferase activity, UDP-glucose:nicotinate N-glucosyltransferase activity, UDP-glucose:nicotinic acid-N-glucosyltransferase activity, UDPglucose:nicotinate N-glucosyltransferase activity, uridine diphosphoglucose-nicotinate N-glucosyltransferase activity